{
  "term_id": "GO:0005737",
  "gene_symbol": "GNPDA2",
  "gene_name": "Glucosamine-6-phosphate isomerase 2",
  "gene": "UniProtKB:Q8TDQ7",
  "term_label": "cytoplasm"
}